{
  "term_id": "GO:0005634",
  "term_label": "nucleus",
  "gene_name": "DNA repair and recombination protein RAD54B",
  "gene": "UniProtKB:Q9Y620",
  "gene_symbol": "RAD54B"
}